{
  "gene_name": "Echinoderm microtubule-associated protein-like 1",
  "term_label": "microtubule binding",
  "term_id": "GO:0008017",
  "gene_symbol": "EML1",
  "gene": "UniProtKB:O00423"
}